{
  "gene": "UniProtKB:Q8WXF5",
  "gene_name": "Gamma-crystallin N",
  "gene_symbol": "CRYGN",
  "term_label": "Unknown cellular component",
  "term_id": "UNKNOWN:0003"
}